{
  "gene_name": "Phosphatidate cytidylyltransferase 1",
  "term_id": "GO:0016024",
  "term_label": "CDP-diacylglycerol biosynthetic process",
  "gene": "UniProtKB:Q92903",
  "gene_symbol": "CDS1"
}